{
  "term_label": "Unknown molecular function",
  "gene_symbol": "C19orf25",
  "gene": "UniProtKB:Q9UFG5",
  "term_id": "UNKNOWN:0001",
  "gene_name": "UPF0449 protein C19orf25"
}